{
  "gene": "UniProtKB:Q9ULX6",
  "term_id": "GO:0007076",
  "gene_name": "A-kinase anchor protein 8-like",
  "term_label": "mitotic chromosome condensation",
  "gene_symbol": "AKAP8L"
}